mitotic M phase [GO:0000087] (biological process) Also known as: M phase of mitotic cell cycle, M-phase of mitotic cell cycle Subtypes: mitotic prometaphase [GO:0000236] Relationships: is_a M phase [GO:0000279]; is a type of mitotic cell cycle phase [GO:0098763] Definition: A cell cycle phase during which nuclear division occurs, and which is comprises the phases: prophase, metaphase, anaphase and telophase and occurs as part of a mitotic cell cycle. Note: Note that this term should not be used for direct annotation. If you are trying to make an annotation to x phase, it is likely that the correct annotation is 'regulation of x/y phase transition' or to a process which occurs during the reported phase (i.e mitotic DNA replication for mitotic S-phase). To capture the phase when a specific location or process is observed, the phase term can be used in an annotation extension (PMID:24885854) applied to a cellular component term (with the relation exists_during) or a biological process term (with the relation happens_during). Sources: GOC:mtg_cell_cycle